{
  "gene": "UniProtKB:Q7Z494",
  "gene_name": "Nephrocystin-3",
  "gene_symbol": "NPHP3",
  "term_label": "ciliary base",
  "term_id": "GO:0097546"
}